{
  "gene_symbol": "RXFP1",
  "term_id": "GO:0008528",
  "gene_name": "Relaxin receptor 1",
  "gene": "UniProtKB:Q9HBX9",
  "term_label": "G protein-coupled peptide receptor activity"
}